{
  "term_id": "GO:0004128",
  "gene": "UniProtKB:Q7L1T6",
  "term_label": "cytochrome-b5 reductase activity, acting on NAD(P)H",
  "gene_symbol": "CYB5R4",
  "gene_name": "Cytochrome b5 reductase 4"
}